coronary vasculature development [GO:0060976] (biological process) Also known as: cardiac blood vessel development, cardiac vasculature development, coronary blood vessel development, heart blood vessel development, heart vasculature development Sources: GOC:mtg_heart Definition: The process whose specific outcome is the progression of the blood vessels of the heart over time, from its formation to the mature structure. Relationships: is a type of blood vessel development [GO:0001568]; is part of GO:0007507